sphingolipid catabolic process [GO:0030149] (biological process) Subtypes: sphingomyelin catabolic process [GO:0006685], glycosphingolipid catabolic process [GO:0046479], ceramide catabolic process [GO:0046514], sphingoid catabolic process [GO:0046521], sphinganine-1-phosphate catabolic process [GO:0051874], ceramide phosphoethanolamine catabolic process [GO:1905372] Sources: GOC:mah, ISBN:0198506732 Definition: The chemical reactions and pathways resulting in the breakdown of sphingolipids, any of a class of lipids containing the long-chain amine diol sphingosine or a closely related base (a sphingoid). Relationships: is a type of sphingolipid metabolic process [GO:0006665]; is_a GO:0046466 Also known as: sphingolipid breakdown, sphingolipid catabolism, sphingolipid degradation